{
  "term_id": "GO:0070828",
  "term_label": "heterochromatin organization",
  "gene_name": "Heterochromatin protein 1-binding protein 3",
  "gene_symbol": "HP1BP3",
  "gene": "UniProtKB:Q5SSJ5"
}